{
  "gene": "UniProtKB:P30518",
  "term_label": "regulation of systemic arterial blood pressure by vasopressin",
  "gene_name": "Vasopressin V2 receptor",
  "gene_symbol": "AVPR2",
  "term_id": "GO:0001992"
}